{
  "gene_name": "Transmembrane and immunoglobulin domain-containing protein 2",
  "term_label": "Unknown biological process",
  "term_id": "UNKNOWN:0002",
  "gene_symbol": "TMIGD2",
  "gene": "UniProtKB:Q96BF3"
}